{
  "term_id": "GO:0002283",
  "gene_name": "Tyrosine-protein kinase SYK",
  "term_label": "neutrophil activation involved in immune response",
  "gene": "UniProtKB:P43405",
  "gene_symbol": "SYK"
}